{
  "term_id": "GO:0045776",
  "gene_name": "Nitric oxide synthase, inducible",
  "gene_symbol": "NOS2",
  "term_label": "negative regulation of blood pressure",
  "gene": "UniProtKB:P35228"
}